positive regulation of transport across blood-brain barrier [GO:0150201] (biological process) Definition: Any process that activates or increases the frequency, rate or extent of transport across blood-brain barrier. References: PMID:29377008, PMID:30280653 Sources: GOC:aruk, GOC:bc Subtypes: positive regulation of lipid transport across blood-brain barrier [GO:1903002] Relationships: is a type of positive regulation of transport [GO:0051050]; is a type of GO:0051240; is a type of regulation of transport across blood-brain barrier [GO:0150200]; is part of GO:0043117; positively regulates transport across blood-brain barrier [GO:0150104]